{
  "gene_symbol": "FAM90A23",
  "term_label": "Unknown cellular component",
  "gene": "UniProtKB:A8MXZ1",
  "gene_name": "Putative protein FAM90A23",
  "term_id": "UNKNOWN:0003"
}